{
  "gene_name": "Sodium channel subunit beta-1",
  "gene_symbol": "SCN1B",
  "term_id": "GO:0044325",
  "term_label": "transmembrane transporter binding",
  "gene": "UniProtKB:Q07699"
}